{
  "gene_name": "Polyisoprenoid diphosphate_phosphate phosphohydrolase PLPP6",
  "gene": "UniProtKB:Q8IY26",
  "term_id": "GO:0016020",
  "term_label": "membrane",
  "gene_symbol": "PLPP6"
}